{
  "term_id": "GO:0004782",
  "term_label": "sulfinoalanine decarboxylase activity",
  "gene_symbol": "CSAD",
  "gene": "UniProtKB:Q9Y600",
  "gene_name": "Cysteine sulfinic acid decarboxylase"
}